{
  "gene": "UniProtKB:Q9HCP0",
  "gene_symbol": "CSNK1G1",
  "gene_name": "Casein kinase I isoform gamma-1",
  "term_id": "GO:0007165",
  "term_label": "signal transduction"
}